{
  "term_id": "GO:0045202",
  "gene_symbol": "CDHR5",
  "term_label": "synapse",
  "gene": "UniProtKB:Q9HBB8",
  "gene_name": "Cadherin-related family member 5"
}